{
  "term_id": "GO:0005829",
  "gene_name": "BTB_POZ domain-containing protein 2",
  "term_label": "cytosol",
  "gene_symbol": "BTBD2",
  "gene": "UniProtKB:Q9BX70"
}